{
  "gene_symbol": "ATP13A4",
  "term_label": "late endosome membrane",
  "gene_name": "Probable cation-transporting ATPase 13A4",
  "gene": "UniProtKB:Q4VNC1",
  "term_id": "GO:0031902"
}